cellular response to thyroxine stimulus [GO:0097069] (biological process) Relationships: is a type of cellular response to amino acid stimulus [GO:0071230]; is a type of cellular response to thyroid hormone stimulus [GO:0097067]; is a type of response to thyroxine [GO:0097068]; is a type of cellular response to oxygen-containing compound [GO:1901701]; is a type of cellular response to L-phenylalanine derivative [GO:1904387] References: PMID:9916872 Sources: GOC:sjw Definition: A change in state or activity of a cell (in terms of movement, secretion, enzyme production, gene expression, etc.) as a result of a thyroxine stimulus. Also known as: cellular response to T4 stimulus